{
  "gene_name": "Transmembrane protein 238-like",
  "term_id": "UNKNOWN:0003",
  "term_label": "Unknown cellular component",
  "gene_symbol": "TMEM238L",
  "gene": "UniProtKB:A6NJY4"
}